{
  "term_id": "UNKNOWN:0002",
  "gene_symbol": "LRRC71",
  "gene": "UniProtKB:Q8N4P6",
  "gene_name": "Leucine-rich repeat-containing protein 71",
  "term_label": "Unknown biological process"
}